neural crest cell differentiation involved in thymus development [GO:1902637] (biological process) References: PMID:15741317, PMID:18292542 Sources: GOC:TermGenie, GOC:nhn, GO_REF:0000060 Definition: Any neural crest cell differentiation that is involved in thymus development. Relationships: is a type of neural crest cell differentiation [GO:0014033]; is part of thymus development [GO:0048538]